{
  "term_id": "GO:0060337",
  "gene_symbol": "IFITM2",
  "gene_name": "Interferon-induced transmembrane protein 2",
  "term_label": "type I interferon-mediated signaling pathway",
  "gene": "UniProtKB:Q01629"
}